{
  "term_label": "Unknown molecular function",
  "gene_symbol": "FAM133A",
  "term_id": "UNKNOWN:0001",
  "gene": "UniProtKB:Q8N9E0",
  "gene_name": "Protein FAM133A"
}